{
  "term_id": "GO:0050839",
  "gene": "UniProtKB:Q9Y5G0",
  "gene_symbol": "PCDHGB5",
  "gene_name": "Protocadherin gamma-B5",
  "term_label": "cell adhesion molecule binding"
}